{
  "gene_name": "Regenerating islet-derived protein 3-gamma",
  "gene": "UniProtKB:Q6UW15",
  "term_label": "antimicrobial humoral immune response mediated by antimicrobial peptide",
  "gene_symbol": "REG3G",
  "term_id": "GO:0061844"
}